{
  "gene_symbol": "AURKB",
  "term_id": "GO:0000776",
  "gene_name": "Aurora kinase B",
  "term_label": "kinetochore",
  "gene": "UniProtKB:Q96GD4"
}